dense core granule lumen [GO:0098898] (cellular component) Sources: GOC:dos Also known as: dense core vesicle lumen Definition: The volume enclosed by the dense core granule membrane. Subtypes: neuronal dense core vesicle lumen [GO:0099013] Relationships: is a type of secretory granule lumen [GO:0034774]; is part of dense core granule [GO:0031045]